phosphatidylcholine phospholipase C activity [GO:0034480] (molecular function) Also known as: phospholipase C, acting on phosphatidylcholine, Clostridium oedematiens beta- and gamma-toxins activity, Clostridium welchii alpha-toxin activity, heat-labile hemolysin, lipophosphodiesterase I activity, phosphatidylcholine cholinephosphohydrolase activity Definition: Catalysis of the reaction: a 1,2-diacyl-sn-glycero-3-phosphocholine + H2O = a 1,2-diacyl-sn-glycerol + H+ + phosphocholine. Relationships: is_a phospholipase C activity [GO:0004629] Sources: GOC:mah, RHEA:10604